{
  "term_label": "Unknown biological process",
  "gene_symbol": "UBALD2",
  "term_id": "UNKNOWN:0002",
  "gene_name": "UBA-like domain-containing protein 2",
  "gene": "UniProtKB:Q8IYN6"
}